{
  "term_id": "GO:0003746",
  "gene_symbol": "EEF1A2",
  "gene": "UniProtKB:Q05639",
  "term_label": "translation elongation factor activity",
  "gene_name": "Elongation factor 1-alpha 2"
}